{
  "gene_symbol": "ATRAID",
  "term_id": "UNKNOWN:0001",
  "gene_name": "All-trans retinoic acid-induced differentiation factor",
  "term_label": "Unknown molecular function",
  "gene": "UniProtKB:Q6UW56"
}